{
  "term_id": "GO:0004540",
  "term_label": "RNA nuclease activity",
  "gene": "UniProtKB:P03950",
  "gene_name": "Angiogenin",
  "gene_symbol": "ANG"
}